response to calcium ion [GO:0051592] (biological process) Regulation: regulated by regulation of response to calcium ion [GO:1905945]; negatively regulated by negative regulation of response to calcium ion [GO:1905946]; positively regulated by positive regulation of response to calcium ion [GO:1905947] Also known as: response to Ca2+ ion Definition: Any process that results in a change in state or activity of a cell or an organism (in terms of movement, secretion, enzyme production, gene expression, etc.) as a result of a calcium ion stimulus. Sources: GOC:ai Subtypes: detection of calcium ion [GO:0005513], GO:0071277 Relationships: is a type of GO:0010038